{
  "gene": "UniProtKB:Q8TDW0",
  "gene_symbol": "LRRC8C",
  "term_label": "aspartate transmembrane transport",
  "gene_name": "Volume-regulated anion channel subunit LRRC8C",
  "term_id": "GO:0015810"
}